host cell membrane pore complex [GO:0044084] (cellular component) Sources: MITRE:tk Relationships: is a type of host cell part [GO:0033643]; BFO_0000050 host cell membrane [GO:0033644] Definition: Any small opening in a host cell membrane that allows the passage of gases and/or liquids, composed of host proteins. Also known as: pore complex in host cell membrane